{
  "term_label": "actin filament binding",
  "gene_name": "KICSTOR complex protein kaptin",
  "gene_symbol": "KPTN",
  "term_id": "GO:0051015",
  "gene": "UniProtKB:Q9Y664"
}